regulation of postsynapse organization [GO:0099175] (biological process) Subtypes: regulation of dendritic spine morphogenesis [GO:0061001], regulation of postsynapse assembly [GO:0150052], regulation of dendritic spine maintenance [GO:1902950], regulation of postsynaptic density organization [GO:1905874] Relationships: is a type of regulation of synapse organization [GO:0050807]; regulates postsynapse organization [GO:0099173] Sources: GOC:ai, GOC:dph, GOC:tb Also known as: regulation of postsynapse organisation, regulation of postsynapse structure, regulation of postsynapse organization and biogenesis Definition: Any process that modulates the physical form of a postsynapse.